negative regulation of compound eye retinal cell apoptotic process [GO:1901693] (biological process) References: PMID:12021768 Sources: GOC:TermGenie, GOC:mtg_apoptosis Also known as: down regulation of compound eye retinal cell apoptotic process, down-regulation of compound eye retinal cell apoptotic process, downregulation of compound eye retinal cell apoptotic process, inhibition of compound eye retinal cell apoptotic process Definition: Any process that stops, prevents or reduces the frequency, rate or extent of compound eye retinal cell apoptotic process. Relationships: is a type of negative regulation of apoptotic process [GO:0043066]; is a type of regulation of compound eye retinal cell apoptotic process [GO:1901692]; negatively regulates compound eye retinal cell apoptotic process [GO:1990010]